{
  "gene_name": "Volume-regulated anion channel subunit LRRC8E",
  "term_label": "cytoplasm",
  "gene_symbol": "LRRC8E",
  "gene": "UniProtKB:Q6NSJ5",
  "term_id": "GO:0005737"
}